positive regulation of developmental vegetative growth [GO:1905615] (biological process) Relationships: is a type of positive regulation of developmental growth [GO:0048639]; is a type of regulation of developmental vegetative growth [GO:1905613]; positively regulates developmental vegetative growth [GO:0080186] References: PMID:11606552 Sources: GOC:TermGenie, GO_REF:0000058 Definition: Any process that activates or increases the frequency, rate or extent of developmental vegetative growth. Also known as: up regulation of developmental vegetative growth, up-regulation of developmental vegetative growth, upregulation of developmental vegetative growth, activation of developmental vegetative growth